{
  "gene_name": "Engulfment and cell motility protein 2",
  "term_id": "GO:2001212",
  "term_label": "regulation of vasculogenesis",
  "gene": "UniProtKB:Q96JJ3",
  "gene_symbol": "ELMO2"
}